glycerophospholipid metabolic process [GO:0006650] (biological process) Definition: The chemical reactions and pathways involving glycerophospholipids, any derivative of glycerophosphate that contains at least one O-acyl, O-alkyl, or O-alkenyl group attached to the glycerol residue. Sources: ISBN:0198506732 Also known as: glycerophospholipid metabolism, phosphoglyceride metabolic process, phosphoglyceride metabolism, alpha-glycerophosphate pathway Relationships: is a type of phospholipid metabolic process [GO:0006644]; is a type of glycerolipid metabolic process [GO:0046486] Subtypes: phosphatidylserine metabolic process [GO:0006658], phosphatidylethanolamine metabolic process [GO:0046337], GO:0046341, platelet activating factor metabolic process [GO:0046469], phosphatidylcholine metabolic process [GO:0046470], phosphatidylglycerol metabolic process [GO:0046471], phosphatidic acid metabolic process [GO:0046473], GO:0046474, glycerophospholipid catabolic process [GO:0046475], phosphatidylinositol metabolic process [GO:0046488], GO:2001311